{
  "gene": "UniProtKB:P09619",
  "term_label": "angiogenesis",
  "gene_name": "Platelet-derived growth factor receptor beta",
  "gene_symbol": "PDGFRB",
  "term_id": "GO:0001525"
}